{
  "gene": "UniProtKB:Q02413",
  "term_id": "GO:0005509",
  "gene_symbol": "DSG1",
  "term_label": "calcium ion binding",
  "gene_name": "Desmoglein-1"
}